{
  "gene_symbol": "MTMR7",
  "term_id": "GO:0004438",
  "gene_name": "Myotubularin-related protein 7",
  "gene": "UniProtKB:Q9Y216",
  "term_label": "phosphatidylinositol-3-phosphate phosphatase activity"
}